{
  "gene_symbol": "SERGEF",
  "term_label": "cytoplasm",
  "gene": "UniProtKB:Q9UGK8",
  "term_id": "GO:0005737",
  "gene_name": "Secretion-regulating guanine nucleotide exchange factor"
}